{
  "gene_symbol": "ZNF287",
  "gene": "UniProtKB:Q9HBT7",
  "gene_name": "Zinc finger protein 287",
  "term_id": "GO:0006357",
  "term_label": "regulation of transcription by RNA polymerase II"
}